{
  "gene": "UniProtKB:Q5JSZ5",
  "term_label": "Unknown cellular component",
  "gene_name": "Protein PRRC2B",
  "gene_symbol": "PRRC2B",
  "term_id": "UNKNOWN:0003"
}